G protein-coupled acetylcholine receptor signaling pathway involved in negative regulation of heart rate [GO:0086033] (biological process) Definition: A G protein-coupled acetylcholine receptor signaling pathway that contributes to a decrease in frequency or rate of heart contraction. Binding of acetylcholine to a G protein-coupled (muscarinic) receptor on the surface of the signal-receiving cell results in the alpha subunit of a coupled G-protein binding to GTP. This results in the separation of the beta-gamma complex from the alpha subunit. Both the alpha subunit, and the beta-gamma complex can continue to signal to bring about membrane hyperpolarization and a reduction in heart rate. Sources: GOC:BHF, GOC:mtg_cardiac_conduct_nov11, Wikipedia:G_protein-gated_ion_channel Relationships: is a type of G protein-coupled acetylcholine receptor signaling pathway involved in heart process [GO:0086093]; is part of negative regulation of heart rate by acetylcholine [GO:0003063] Also known as: G-protein coupled acetylcholine receptor signaling pathway involved in negative regulation of heart rate, M2 receptor signalling pathway involved in negative regulation of heart rate, muscarinic acetylcholine receptor signaling pathway involved in negative regulation of heart rate, muscarinic receptor signalling pathway involved in negative regulation of heart rate